{
  "term_label": "ribosome binding",
  "gene": "UniProtKB:P61619",
  "gene_name": "Protein transport protein Sec61 subunit alpha isoform 1",
  "gene_symbol": "SEC61A1",
  "term_id": "GO:0043022"
}